{
  "term_id": "GO:0045892",
  "gene": "UniProtKB:Q96PN7",
  "term_label": "negative regulation of DNA-templated transcription",
  "gene_name": "Transcriptional-regulating factor 1",
  "gene_symbol": "TRERF1"
}